ABC-type monosaccharide transporter activity [GO:0015407] (molecular function) Subtypes: ABC-type D-ribose transporter activity [GO:0015611], ABC-type L-arabinose transporter activity [GO:0015612], GO:0015614, ABC-type D-allose transporter activity [GO:0015615], GO:0102014, ABC-type D-galactofuranose transporter [GO:0103116] Relationships: is a type of GO:0015145; is a type of ABC-type carbohydrate transporter activity [GO:0043211] Also known as: ATP-dependent monosaccharide transmembrane transporter activity, monosaccharide-transporting ATPase activity, monosaccharide ABC transporter, monosaccharide-importing ATPase activity, ATPase-coupled monosaccharide transmembrane transporter activity Definition: Enables the transfer of a solute or solutes from one side of a membrane to the other according to the reaction: ATP + H2O + monosaccharide(out) = ADP + phosphate + monosaccharide(in). Ribose, xylose, arabinose, galactose and methylgalactoside are imported. Sources: MetaCyc:3.6.3.17-RXN